{
  "gene_symbol": "FGF8",
  "term_label": "neurogenesis",
  "term_id": "GO:0022008",
  "gene": "UniProtKB:P55075",
  "gene_name": "Fibroblast growth factor 8"
}